{
  "gene_name": "Pantetheinase",
  "term_label": "pantetheine hydrolase activity",
  "gene": "UniProtKB:O95497",
  "term_id": "GO:0017159",
  "gene_symbol": "VNN1"
}